symbiont-mediated suppression of host phytoalexin production [GO:1990217] (biological process) Relationships: is a type of GO:0052165 References: PMID:21402357 Also known as: negative regulation by symbiont of host phytoalexin production, suppression by symbiont of host phytoalexin production Definition: A process in which a symbiont inhibits or disrupts the production of phytoalexins in the host organism. Phytoalexins are produced by plants to fight against pathogens. The host is defined as the larger of the organisms involved in a symbiotic interaction.